{
  "gene_symbol": "MACO1",
  "gene": "UniProtKB:Q8N5G2",
  "term_label": "nuclear membrane",
  "gene_name": "Macoilin",
  "term_id": "GO:0031965"
}